tertiary granule [GO:0070820] (CC) Definition: A secretory granule that contains cathepsin and gelatinase and is readily exocytosed upon cell activation; found primarily in mature neutrophil cells. Relationships: is a type of secretory granule [GO:0030141] References: PMID:12070036 Sources: GOC:BHF, GOC:mah, GOC:rl Also known as: gelatinase granule